fatty aldehyde dehydrogenase (NAD+) activity [GO:0102673] (molecular function) Relationships: is a type of aldehyde dehydrogenase (NAD+) activity [GO:0004029] Also known as: fatty aldehyde dehydrogenase activity Sources: RHEA:49832 Subtypes: long-chain fatty aldehyde dehydrogenase (NAD+) activity [GO:0050061], GO:0052814 Definition: Catalysis of the reaction: a fatty aldehyde + H2O + NAD+ = a fatty acid + 2 H+ + NADH.